{
  "gene": "UniProtKB:A2VEC9",
  "gene_name": "SCO-spondin",
  "term_id": "GO:0005201",
  "gene_symbol": "SSPOP",
  "term_label": "extracellular matrix structural constituent"
}